6-hydroxyhexanoate dehydrogenase activity [GO:0018463] (molecular function) Also known as: 6-hydroxyhexanoate:NAD+ oxidoreductase activity Relationships: is a type of oxidoreductase activity, acting on the CH-OH group of donors, NAD or NADP as acceptor [GO:0016616] Definition: Catalysis of the reaction: 6-hydroxyhexanoate + NAD+ = 6-oxohexanoate + H+ + NADH. Sources: EC:1.1.1.258, RHEA:14225